{
  "gene_symbol": "USP46",
  "term_label": "cysteine-type deubiquitinase activity",
  "gene_name": "Ubiquitin carboxyl-terminal hydrolase 46",
  "gene": "UniProtKB:P62068",
  "term_id": "GO:0004843"
}